{
  "term_id": "GO:0031267",
  "term_label": "small GTPase binding",
  "gene_name": "Rab GTPase-activating protein 1-like",
  "gene": "UniProtKB:Q5R372",
  "gene_symbol": "RABGAP1L"
}